{
  "gene": "UniProtKB:Q9NRW3",
  "term_id": "GO:0016554",
  "term_label": "cytidine to uridine editing",
  "gene_name": "DNA dC-dU-editing enzyme APOBEC-3C",
  "gene_symbol": "APOBEC3C"
}